{
  "gene_symbol": "FBXL20",
  "gene_name": "F-box_LRR-repeat protein 20",
  "gene": "UniProtKB:Q96IG2",
  "term_label": "SCF ubiquitin ligase complex",
  "term_id": "GO:0019005"
}